regulation of mitochondrial translational elongation [GO:1905082] (biological process) References: PMID:25738458 Sources: GOC:TermGenie, GO_REF:0000058 Definition: Any process that modulates the frequency, rate or extent of mitochondrial translational elongation. Relationships: is a type of regulation of translational elongation [GO:0006448]; RO_0002211 mitochondrial translational elongation [GO:0070125] Subtypes: negative regulation of mitochondrial translational elongation [GO:1905083], positive regulation of mitochondrial translational elongation [GO:1905084] Also known as: regulation of mitochondrial translation elongation